{
  "term_label": "plasma membrane",
  "gene_symbol": "KCNJ9",
  "term_id": "GO:0005886",
  "gene": "UniProtKB:Q92806",
  "gene_name": "G protein-activated inward rectifier potassium channel 3"
}